sulfur compound biosynthetic process [GO:0044272] (BP) Subtypes: sulfur amino acid biosynthetic process [GO:0000097], L-methionine catabolic process to 3-methylthiopropanol [GO:0000951], GO:0000954, S-adenosylmethionine biosynthetic process [GO:0006556], glutathione biosynthetic process [GO:0006750], biotin biosynthetic process [GO:0009102], lipoate biosynthetic process [GO:0009107], GO:0010120, mycothiol biosynthetic process [GO:0010125], GO:0010250, GO:0015937, S-glycoside biosynthetic process [GO:0016144], coenzyme M biosynthetic process [GO:0019295], penicillin biosynthetic process [GO:0042318], GO:0042724, pyochelin biosynthetic process [GO:0042864], GO:0043646, GO:0046305, GO:0046506, GO:0048107, 3'-phosphoadenosine 5'-phosphosulfate biosynthetic process [GO:0050428], epothilone biosynthetic process [GO:0050814], thiazole biosynthetic process [GO:0052837], GO:0070814, acyl-CoA biosynthetic process [GO:0071616], GO:0071793, cephamycin C biosynthetic process [GO:1901118], glutathione derivative biosynthetic process [GO:1901687], leukotriene D4 biosynthetic process [GO:1901750], GO:2001310 Relationships: is_a GO:0006790; is a type of biosynthetic process [GO:0009058] Also known as: sulfur compound anabolism, sulfur compound biosynthesis, sulfur compound formation, sulfur compound synthesis, sulfur biosynthesis, sulfur biosynthetic process Definition: The chemical reactions and pathways resulting in the formation of compounds that contain sulfur, such as the amino acids methionine and cysteine or the tripeptide glutathione. Sources: GOC:jl